{
  "term_label": "cell adhesion molecule binding",
  "term_id": "GO:0050839",
  "gene": "UniProtKB:Q8N0Z9",
  "gene_name": "V-set and immunoglobulin domain-containing protein 10",
  "gene_symbol": "VSIG10"
}